ventral aorta development [GO:0035908] (BP) Definition: The progression of the ventral aorta over time, from its initial formation to the mature structure. The ventral aorta is a blood vessel in a single-pass circulatory system that carries de-oxygenated blood from the heart to the gills. In a single-pass circulatory system blood passes once through the heart to supply the body once. Sources: GOC:bf, GOC:dgh, UBERON:0003085, Wikipedia:Aorta, ZFA:0000604 Relationships: is_a GO:0035904